{
  "gene_name": "Ubiquitin-associated and SH3 domain-containing protein A",
  "gene": "UniProtKB:P57075",
  "gene_symbol": "UBASH3A",
  "term_label": "cytoplasm",
  "term_id": "GO:0005737"
}